positive regulation of mesenchymal to epithelial transition involved in mesonephros morphogenesis [GO:2000086] (biological process) Also known as: positive regulation of mesonephric mesenchyme to epithelial transition Sources: GOC:mtg_kidney_jan10 Definition: Any process that activates or increases the frequency, rate or extent of mesenchymal to epithelial transition involved in mesonephros morphogenesis. Relationships: is a type of GO:2000084; is a type of positive regulation of epithelial cell differentiation involved in kidney development [GO:2000698]; positively regulates mesenchymal to epithelial transition involved in mesonephros morphogenesis [GO:0061261]